{
  "term_label": "Unknown cellular component",
  "gene": "UniProtKB:Q9XRX5",
  "gene_name": "HERV-H LTR-associating protein 3",
  "gene_symbol": "HHLA3",
  "term_id": "UNKNOWN:0003"
}